{
  "gene_name": "BTB_POZ domain-containing adapter for CUL3-mediated RhoA degradation protein 2",
  "term_id": "GO:0043161",
  "term_label": "proteasome-mediated ubiquitin-dependent protein catabolic process",
  "gene": "UniProtKB:Q13829",
  "gene_symbol": "TNFAIP1"
}